potassium channel activator activity [GO:0099104] (molecular function) Relationships: is a type of potassium channel regulator activity [GO:0015459]; is a type of channel activator activity [GO:0099103]; positively regulates potassium channel activity [GO:0005267] Sources: GOC:dos Definition: Binds to and increases the activity of a potassium channel, resulting in its opening.